snRNA 2'-O-methylation [GO:1990437] (biological process) Definition: The posttranscriptional addition of a methyl group to the 2' oxygen atom of a nucleotide residue in an snRNA molecule. Relationships: is a type of snRNA methylation [GO:0106349] References: PMID:11842100, PMID:9844635 Subtypes: GO:1990438